glutarate-CoA ligase activity [GO:0047948] (molecular function) Also known as: glutarate:CoA ligase (ADP-forming), glutaryl coenzyme A synthetase activity, glutaryl-CoA synthetase activity Definition: Catalysis of the reaction: ATP + CoA + glutarate = ADP + glutaryl-CoA + H+ + phosphate. Sources: EC:6.2.1.6, RHEA:14169 Relationships: is a type of acid-thiol ligase activity [GO:0016878]